{
  "gene_symbol": "KCNK17",
  "term_id": "GO:0005886",
  "gene_name": "Potassium channel subfamily K member 17",
  "gene": "UniProtKB:Q96T54",
  "term_label": "plasma membrane"
}